{
  "term_label": "regulation of platelet activation",
  "gene": "UniProtKB:P04196",
  "gene_symbol": "HRG",
  "term_id": "GO:0010543",
  "gene_name": "Histidine-rich glycoprotein"
}